tubulin deacetylation [GO:0090042] (biological process) Regulation: regulated by regulation of tubulin deacetylation [GO:0090043]; positively regulated by positive regulation of tubulin deacetylation [GO:0090044]; negatively regulated by GO:1904428 Definition: The removal of an acetyl group from tubulin. An acetyl group is CH3CO-, derived from acetic [ethanoic] acid. Sources: GOC:BHF, GOC:dph, GOC:tb Relationships: is a type of protein deacetylation [GO:0006476]